establishment of proximal/distal cell polarity [GO:0022606] (biological process) Definition: The specification and formation of the polarity of a cell along its proximal/distal axis. Relationships: is a type of establishment of monopolar cell polarity [GO:0061162] Sources: GOC:isa_complete Subtypes: imaginal disc-derived wing hair site selection [GO:0035320]